pyridoxamine metabolic process [GO:0042818] (biological process) Sources: GOC:jl Definition: The chemical reactions and pathways involving 4-(aminomethyl)-5-(hydroxymethyl)-2-methylpyridin-3-ol, one of the vitamin B6 compounds. Pyridoxal, pyridoxamine and pyridoxine are collectively known as vitamin B6, and are efficiently converted to the biologically active form of vitamin B6, pyridoxal phosphate. Relationships: is a type of vitamin B6 metabolic process [GO:0042816] Also known as: pyridoxamine metabolism Subtypes: pyridoxal phosphate biosynthetic process from pyridoxamine [GO:0010144]